{
  "term_label": "cilium",
  "term_id": "GO:0005929",
  "gene_name": "Nephrocystin-1",
  "gene": "UniProtKB:O15259",
  "gene_symbol": "NPHP1"
}